{
  "gene_name": "Nonsense-mediated mRNA decay factor SMG5",
  "term_id": "GO:0005697",
  "gene_symbol": "SMG5",
  "gene": "UniProtKB:Q9UPR3",
  "term_label": "telomerase holoenzyme complex"
}